{
  "gene": "UniProtKB:Q9NQL9",
  "term_id": "GO:0007548",
  "term_label": "sex differentiation",
  "gene_symbol": "DMRT3",
  "gene_name": "Doublesex- and mab-3-related transcription factor 3"
}